{
  "term_id": "GO:0006935",
  "gene_name": "Ras-related C3 botulinum toxin substrate 2",
  "gene_symbol": "RAC2",
  "gene": "UniProtKB:P15153",
  "term_label": "chemotaxis"
}